osteoclast proliferation [GO:0002158] (biological process) Regulation: regulated by regulation of osteoclast proliferation [GO:0090289]; RO_0002213 by positive regulation of osteoclast proliferation [GO:0090290]; negatively regulated by negative regulation of osteoclast proliferation [GO:0090291] Sources: CL:0000092, GOC:hjd Relationships: is a type of leukocyte proliferation [GO:0070661] Definition: The multiplication or reproduction of osteoclasts, resulting in the expansion of an osteoclast cell population. An osteoclast is a specialized phagocytic cell associated with the absorption and removal of the mineralized matrix of bone tissue, which typically differentiates from monocytes.